{
  "term_id": "UNKNOWN:0002",
  "gene_symbol": "TPST1",
  "term_label": "Unknown biological process",
  "gene": "UniProtKB:O60507",
  "gene_name": "Protein-tyrosine sulfotransferase 1"
}